{
  "gene": "UniProtKB:O95302",
  "gene_name": "Peptidyl-prolyl cis-trans isomerase FKBP9",
  "term_label": "endoplasmic reticulum",
  "gene_symbol": "FKBP9",
  "term_id": "GO:0005783"
}